feeding behavior [GO:0007631] (biological process) Regulation: regulated by regulation of feeding behavior [GO:0060259]; negatively regulated by negative regulation of feeding behavior [GO:2000252]; RO_0002213 by positive regulation of feeding behavior [GO:2000253] Note: See also the biological process term 'behavior ; GO:0007610'. Definition: Behavior associated with the intake of food. Sources: GOC:mah Subtypes: conditioned taste aversion [GO:0001661], suckling behavior [GO:0001967], GO:0008343, larval feeding behavior [GO:0030536], salt aversion [GO:0035199], eating behavior [GO:0042755], GO:0042756, GO:0140106 Relationships: is a type of behavior [GO:0007610] Also known as: behavioral response to food, behavioural response to food, feeding behaviour, eating, feeding from phloem of other organism, feeding from plant phloem, feeding from tissue of other organism, feeding from vascular tissue of another organism, feeding from xylem of other organism, feeding on or from other organism, feeding on plant sap